{
  "gene_name": "Dihydrolipoyllysine-residue acetyltransferase component of pyruvate dehydrogenase complex, mitochondrial",
  "term_id": "GO:0004742",
  "term_label": "dihydrolipoyllysine-residue acetyltransferase activity",
  "gene_symbol": "DLAT",
  "gene": "UniProtKB:P10515"
}